{
  "gene": "UniProtKB:O43638",
  "gene_symbol": "FOXS1",
  "gene_name": "Forkhead box protein S1",
  "term_id": "UNKNOWN:0003",
  "term_label": "Unknown cellular component"
}